{
  "gene": "UniProtKB:Q9BW11",
  "gene_name": "Max dimerization protein 3",
  "gene_symbol": "MXD3",
  "term_id": "GO:0000978",
  "term_label": "RNA polymerase II cis-regulatory region sequence-specific DNA binding"
}